COPI-coated vesicle budding [GO:0035964] (biological process) Relationships: is a type of vesicle budding from membrane [GO:0006900]; is part of GO:0048199 Also known as: COPI vesicle budding References: PMID:10052452, PMID:17041781 Sources: GOC:br Definition: The evagination of a Golgi membrane, resulting in formation of a COPI-coated vesicle.